diacylglycerol binding [GO:0019992] (molecular function) Relationships: is a type of lipid binding [GO:0008289] Definition: Binding to a diacylglycerol, a diester of glycerol and two fatty acids. Sources: GOC:ma